acetylcholine receptor activator activity [GO:0030549] (MF) Sources: GOC:mah Relationships: is a type of signaling receptor activator activity [GO:0030546]; is a type of GO:0030548; RO_0002213 acetylcholine receptor activity [GO:0015464] Definition: Interacting (directly or indirectly) with acetylcholine receptors such that the proportion of receptors in the active form is increased.